{
  "term_id": "GO:0002040",
  "term_label": "sprouting angiogenesis",
  "gene": "UniProtKB:O43915",
  "gene_symbol": "VEGFD",
  "gene_name": "Vascular endothelial growth factor D"
}